{
  "gene": "UniProtKB:Q9NWM0",
  "term_id": "GO:0005737",
  "term_label": "cytoplasm",
  "gene_name": "Spermine oxidase",
  "gene_symbol": "SMOX"
}